{
  "gene_symbol": "ART1",
  "gene": "UniProtKB:P52961",
  "term_id": "UNKNOWN:0002",
  "term_label": "Unknown biological process",
  "gene_name": "GPI-linked NAD(P)(+)--arginine ADP-ribosyltransferase 1"
}